{
  "term_label": "centrosome cycle",
  "gene_symbol": "CEP192",
  "gene_name": "Centrosomal protein of 192 kDa",
  "gene": "UniProtKB:Q8TEP8",
  "term_id": "GO:0007098"
}